{
  "term_id": "UNKNOWN:0001",
  "term_label": "Unknown molecular function",
  "gene_symbol": "TRAJ54",
  "gene_name": "T cell receptor alpha joining 54 (Fragment)",
  "gene": "UniProtKB:A0A075B712"
}